genital disc sexually dimorphic development [GO:0035263] (biological process) Definition: The sex-specific patterns of primoridia growth and differentiation in the genital imaginal disc. The anal primordium of the genital disc develops in both sexes, but depending on the genetic sex gives rise to either male or female analia. Depending on the genetic sex, only one of the two genital primordia develop. In females the female genital primordium develops and gives rise to the female genitalia whereas the male primordium is repressed. Conversely, in males the male genital primordium develops and gives rise to the male genitalia whereas the female genital primordium is repressed. Relationships: is a type of developmental process involved in reproduction [GO:0003006]; is a type of multicellular organismal reproductive process [GO:0048609]; is part of sex differentiation [GO:0007548]; is part of genital disc development [GO:0035215] References: PMID:11290302, PMID:11494318, PMID:11702781